{
  "gene_symbol": "PLA2G2A",
  "term_id": "GO:0005509",
  "gene_name": "Phospholipase A2, membrane associated",
  "term_label": "calcium ion binding",
  "gene": "UniProtKB:P14555"
}